capsanthin catabolic process [GO:1901808] (BP) Definition: The chemical reactions and pathways resulting in the breakdown of capsanthin. References: PMID:10995282 Sources: GOC:TermGenie, GOC:yaf, UniPathway:UPA00806 Also known as: capsanthin breakdown, capsanthin catabolism, capsanthin degradation Relationships: is a type of GO:0016124